positive regulation of sodium ion import across plasma membrane [GO:1903784] (BP) Definition: Any process that activates or increases the frequency, rate or extent of sodium ion import across the plasma membrane. References: PMID:19376779 Sources: GOC:BHF, GOC:TermGenie, GOC:mtg_cardiac_conduct_nov11, GOC:nc, GO_REF:0000058 Also known as: up regulation of sodium ion import across plasma membrane, up-regulation of sodium ion import across plasma membrane, upregulation of sodium ion import across plasma membrane, activation of sodium ion import across plasma membrane Relationships: is a type of GO:1902307; is a type of regulation of sodium ion import across plasma membrane [GO:1903782]; positively regulates sodium ion import across plasma membrane [GO:0098719]